{
  "term_label": "interleukin-12 receptor binding",
  "gene_symbol": "IL23R",
  "term_id": "GO:0005143",
  "gene": "UniProtKB:Q5VWK5",
  "gene_name": "Interleukin-23 receptor"
}